{
  "term_label": "DNA-binding transcription factor activity, RNA polymerase II-specific",
  "gene_symbol": "MAF",
  "term_id": "GO:0000981",
  "gene_name": "Transcription factor Maf",
  "gene": "UniProtKB:O75444"
}